{
  "term_label": "Unknown cellular component",
  "gene": "UniProtKB:Q8WTU2",
  "term_id": "UNKNOWN:0003",
  "gene_name": "Scavenger receptor cysteine-rich domain-containing group B protein",
  "gene_symbol": "SSC4D"
}